{
  "gene_symbol": "IL6ST",
  "term_label": "cytokine binding",
  "term_id": "GO:0019955",
  "gene_name": "Interleukin-6 receptor subunit beta",
  "gene": "UniProtKB:P40189"
}